{
  "gene": "UniProtKB:Q9UK11",
  "gene_symbol": "ZNF223",
  "term_id": "UNKNOWN:0003",
  "gene_name": "Zinc finger protein 223",
  "term_label": "Unknown cellular component"
}